{
  "term_label": "nuclear exosome (RNase complex)",
  "gene": "UniProtKB:Q9NQT4",
  "gene_symbol": "EXOSC5",
  "gene_name": "Exosome complex component RRP46",
  "term_id": "GO:0000176"
}